{
  "gene_symbol": "GPR84",
  "gene": "UniProtKB:Q9NQS5",
  "gene_name": "G-protein coupled receptor 84",
  "term_id": "GO:0005886",
  "term_label": "plasma membrane"
}